{
  "gene_name": "Glutamate-rich protein 5",
  "gene_symbol": "ERICH5",
  "term_label": "Unknown biological process",
  "term_id": "UNKNOWN:0002",
  "gene": "UniProtKB:Q6P6B1"
}